{
  "gene_name": "Autoimmune regulator",
  "gene": "UniProtKB:O43918",
  "term_id": "GO:0006959",
  "term_label": "humoral immune response",
  "gene_symbol": "AIRE"
}